{
  "term_label": "DNA-binding transcription factor activity, RNA polymerase II-specific",
  "gene_symbol": "ZNF883",
  "gene_name": "Zinc finger protein 883",
  "gene": "UniProtKB:P0CG24",
  "term_id": "GO:0000981"
}